primary neural tube formation [GO:0014020] (biological process) Also known as: primary neural tube morphogenesis, primary neurulation, neural rod cavitation References: PMID:15327780 Sources: GOC:ef, ISBN:0878932585 Relationships: is a type of embryonic epithelial tube formation [GO:0001838]; is part of GO:0001841 Definition: The formation of the neural tube from an epithelial cell sheet (the neuroepithelium or neural plate). In primary neurulation, the cells surrounding the neural plate direct the neural plate cells to proliferate, invaginate, and pinch off from the surface to form a hollow epithelial tube. Primary neurulation is the typical mechanism of formation of the anterior neural tube.